{
  "term_label": "Unknown molecular function",
  "gene": "UniProtKB:A0A1B0GU71",
  "gene_symbol": "CFAP97D2",
  "term_id": "UNKNOWN:0001",
  "gene_name": "Uncharacterized protein CFAP97D2"
}